response to low fluence red light stimulus [GO:0010202] (biological process) Relationships: is a type of response to low light intensity stimulus [GO:0009645]; is a type of response to red light [GO:0010114] Definition: Any process that results in a change in state or activity of a cell or an organism (in terms of movement, secretion, enzyme production, gene expression, etc.) as a result of a low fluence red light stimulus. Red light is electromagnetic radiation of wavelength of 580-700nm. Low fluence red light is defined in this case as short pulses of red light followed by darkness, providing a light level of 0.001-0.1 mmol/m2/sec. Sources: GOC:mtg_far_red, GOC:sm